{
  "gene_name": "Exosome complex component RRP43",
  "gene": "UniProtKB:Q96B26",
  "term_label": "U5 snRNA 3'-end processing",
  "term_id": "GO:0034476",
  "gene_symbol": "EXOSC8"
}